{
  "term_label": "cytoskeleton",
  "gene": "UniProtKB:Q9NYL9",
  "gene_name": "Tropomodulin-3",
  "gene_symbol": "TMOD3",
  "term_id": "GO:0005856"
}